interleukin-8 receptor activity [GO:0004918] (molecular function) Also known as: IL-8 receptor activity, IL-8R Relationships: is a type of C-X-C chemokine receptor activity [GO:0016494]; is part of interleukin-8-mediated signaling pathway [GO:0038112]; has part GO:0019959 Definition: Combining with interleukin-8 and transmitting the signal from one side of the membrane to the other to initiate a change in cell activity. Sources: GOC:jl, GOC:signaling